2-phenylethylamine receptor activity [GO:1990080] (molecular function) Definition: Combining with the biogenic amine 2-phenylethylamine to initiate a change in cell activity. Also known as: beta-phenylethylamine receptor activity Relationships: is a type of G protein-coupled amine receptor activity [GO:0008227] References: PMID:16878137